{
  "gene_symbol": "COX14",
  "term_id": "GO:0005739",
  "gene": "UniProtKB:Q96I36",
  "term_label": "mitochondrion",
  "gene_name": "Cytochrome c oxidase assembly protein COX14"
}